{
  "gene_name": "Humanin-like 1",
  "gene": "UniProtKB:P0CJ68",
  "term_id": "UNKNOWN:0003",
  "gene_symbol": "MTRNR2L1",
  "term_label": "Unknown cellular component"
}